respiratory chain complex III assembly [GO:0017062] (biological process) Subtypes: mitochondrial respiratory chain complex III assembly [GO:0034551] Also known as: coenzyme Q and cytochrome c reductase complex assembly, coenzyme Q and cytochrome c reductase complex biogenesis, complex III assembly, complex III biogenesis, cytochrome bc(1) complex assembly, cytochrome bc(1) complex biogenesis References: PMID:12833641, PMID:20116362 Sources: GOC:jl Definition: The aggregation, arrangement and bonding together of a set of components to form the cytochrome bc(1) complex, a transmembrane lipoprotein complex that it catalyzes the reduction of cytochrome c by accepting reducing equivalents from Coenzyme Q, by the aggregation, arrangement and bonding together of its constituents. Relationships: is a type of cytochrome complex assembly [GO:0017004]